regulation of B cell deletion [GO:0002867] (biological process) Subtypes: negative regulation of B cell deletion [GO:0002868], positive regulation of B cell deletion [GO:0002869], regulation of central B cell deletion [GO:0002898], regulation of peripheral B cell deletion [GO:0002908] Definition: Any process that modulates the frequency, rate, or extent of B cell deletion. Also known as: regulation of B lymphocyte deletion, regulation of B-cell deletion, regulation of B-lymphocyte deletion Sources: GOC:add Relationships: is a type of regulation of B cell tolerance induction [GO:0002661]; is a type of regulation of B cell apoptotic process [GO:0002902]; is a type of regulation of apoptotic process involved in development [GO:1904748]; regulates GO:0002516